{
  "term_label": "endoplasmic reticulum",
  "term_id": "GO:0005783",
  "gene_name": "Serine_threonine-protein kinase_endoribonuclease IRE1",
  "gene_symbol": "ERN1",
  "gene": "UniProtKB:O75460"
}